N2-(2-carboxyethyl)arginine synthase activity [GO:0033848] (molecular function) Also known as: CEA synthetase activity, CEAS, N2-(2-carboxyethyl)arginine synthetase activity, glyceraldehyde-3-phosphate:L-arginine 2-N-(2-hydroxy-3-oxopropyl) transferase (2-carboxyethyl-forming) activity, glyceraldehyde-3-phosphate:L-arginine N2-(2-hydroxy-3-oxopropyl) transferase (2-carboxyethyl-forming) activity Relationships: is a type of GO:0016765 Definition: Catalysis of the reaction: D-glyceraldehyde 3-phosphate + L-arginine = N(2)-(2-carboxyethyl)-L-arginine + H+ + phosphate. Sources: EC:2.5.1.66, RHEA:10556